{
  "gene_symbol": "YWHAH-AS1",
  "term_id": "UNKNOWN:0001",
  "gene_name": "Putative uncharacterized protein YWHAH-AS1",
  "term_label": "Unknown molecular function",
  "gene": "UniProtKB:Q9Y442"
}